neutral amino acid transmembrane import into vacuole [GO:0034491] (biological process) Definition: The directed movement of neutral amino acids into the vacuole across the vacuolar membrane. Subtypes: GO:0090516, L-valine transmembrane import into vacuole [GO:0110101] Relationships: is a type of neutral amino acid transport [GO:0015804]; is a type of amino acid transmembrane import into vacuole [GO:0032975] Sources: GOC:mah